{
  "term_label": "cytoplasm",
  "gene_symbol": "UCHL1",
  "term_id": "GO:0005737",
  "gene_name": "Ubiquitin carboxyl-terminal hydrolase isozyme L1",
  "gene": "UniProtKB:P09936"
}